chloride transport [GO:0006821] (biological process) Sources: GOC:krc Definition: The directed movement of chloride into, out of or within a cell, or between cells, by means of some agent such as a transporter or pore. Relationships: is a type of monoatomic anion transport [GO:0006820]; is a type of inorganic anion transport [GO:0015698] Subtypes: GO:0030321, chloride transmembrane transport [GO:1902476] Regulation: regulated by GO:2001225; negatively regulated by negative regulation of chloride transport [GO:2001226]